4-aminobenzoate biosynthetic process [GO:0008153] (biological process) Also known as: 4-aminobenzoic acid biosynthesis, 4-aminobenzoic acid biosynthetic process, PABA biosynthesis, PABA biosynthetic process, p-aminobenzoic acid biosynthesis, p-aminobenzoic acid biosynthetic process, para-aminobenzoic acid anabolism, para-aminobenzoic acid biosynthesis, para-aminobenzoic acid biosynthetic process, para-aminobenzoic acid formation, para-aminobenzoic acid synthesis, vitamin Bx biosynthesis, vitamin Bx biosynthetic process Relationships: is_a GO:0008652; is a type of GO:0009073; is a type of GO:0046482; is a type of monocarboxylic acid biosynthetic process [GO:0072330] References: PMID:11377864, PMID:11960743 Sources: ISBN:0198506732, MetaCyc:PWY-6543 Definition: The chemical reactions and pathways resulting in the formation of 4-aminobenzoate, an intermediate in the synthesis of folic acid, a compound which some organisms, e.g. prokaryotes, eukaryotic microbes, and plants, can synthesize de novo. Others, notably mammals, cannot. In yeast, it is present as a factor in the B complex of vitamins.